endoplasmic reticulum-peroxisome tethering [GO:0062095] (BP) Relationships: is a type of peroxisome localization [GO:0060151]; is a type of organelle localization by membrane tethering [GO:0140056] Definition: The attachment of an endoplasmic reticulum membrane to a peroxisome via molecular tethers that physically bridge the two membranes and attach them to each other. References: PMID:28463579